{
  "gene": "UniProtKB:O60936",
  "term_label": "negative regulation of release of cytochrome c from mitochondria",
  "gene_name": "Nucleolar protein 3",
  "gene_symbol": "NOL3",
  "term_id": "GO:0090201"
}